{
  "term_id": "UNKNOWN:0002",
  "term_label": "Unknown biological process",
  "gene": "UniProtKB:Q5HYL7",
  "gene_name": "Transmembrane protein 196",
  "gene_symbol": "TMEM196"
}